appendage morphogenesis [GO:0035107] (biological process) Definition: The process in which the anatomical structures of appendages are generated and organized. An appendage is an organ or part that is attached to the trunk of an organism, such as a limb or a branch. Sources: ISBN:0582227089 Relationships: is a type of anatomical structure morphogenesis [GO:0009653]; is part of appendage development [GO:0048736] Subtypes: fin morphogenesis [GO:0033334], limb morphogenesis [GO:0035108], embryonic appendage morphogenesis [GO:0035113], GO:0035114, GO:0035120, GO:0048800